{
  "gene_symbol": "CETP",
  "term_id": "GO:0046470",
  "term_label": "phosphatidylcholine metabolic process",
  "gene_name": "Cholesteryl ester transfer protein",
  "gene": "UniProtKB:P11597"
}